{
  "gene_symbol": "GRAMD1B",
  "term_label": "intracellular sterol transport",
  "term_id": "GO:0032366",
  "gene": "UniProtKB:Q3KR37",
  "gene_name": "Protein Aster-B"
}